dorsal motor nucleus of vagus nerve development [GO:0021744] (biological process) Sources: GOC:cls, GOC:curators, GOC:dgh, GOC:dph, GOC:jid Relationships: is a type of neural nucleus development [GO:0048857]; is part of medulla oblongata development [GO:0021550] Definition: The process whose specific outcome is the progression of the dorsal motor nucleus of the vagus nerve over time, from its formation to the mature structure.